neurotransmitter:sodium symporter activity [GO:0005328] (molecular function) Definition: Enables the transfer of a solute or solutes from one side of a membrane to the other according to the reaction: neurotransmitter(out) + Na+(out) = neurotransmitter(in) + Na+(in). Relationships: is a type of GO:0005326; is a type of solute:sodium symporter activity [GO:0015370] Sources: TC:2.A.22.-.- Also known as: sodium/neurotransmitter symporter activity